{
  "gene_name": "Pro-epidermal growth factor",
  "term_id": "GO:0007173",
  "gene_symbol": "EGF",
  "gene": "UniProtKB:P01133",
  "term_label": "epidermal growth factor receptor signaling pathway"
}